phenylacetyl-CoA hydrolase activity [GO:0033880] (MF) Relationships: is a type of acyl-CoA hydrolase activity [GO:0016289] Definition: Catalysis of the reaction: H2O + phenylglyoxylyl-CoA = CoA + H+ + phenylglyoxylate. Sources: EC:3.1.2.25, RHEA:15337 Also known as: phenylglyoxylyl-CoA hydrolase activity